{
  "term_label": "protein stabilization",
  "gene_name": "Protein Mdm4",
  "gene_symbol": "MDM4",
  "term_id": "GO:0050821",
  "gene": "UniProtKB:O15151"
}